{
  "term_id": "GO:0030121",
  "gene_symbol": "CLBA1",
  "gene_name": "Uncharacterized protein CLBA1",
  "gene": "UniProtKB:Q96F83",
  "term_label": "AP-1 adaptor complex"
}